{
  "gene_name": "Cadherin-17",
  "term_label": "adherens junction",
  "term_id": "GO:0005912",
  "gene": "UniProtKB:Q12864",
  "gene_symbol": "CDH17"
}